{
  "term_id": "GO:0030863",
  "gene_name": "F-actin-capping protein subunit alpha-2",
  "gene_symbol": "CAPZA2",
  "term_label": "cortical cytoskeleton",
  "gene": "UniProtKB:P47755"
}